{
  "term_label": "guanyl-nucleotide exchange factor activity",
  "gene": "UniProtKB:Q14C86",
  "term_id": "GO:0005085",
  "gene_symbol": "GAPVD1",
  "gene_name": "GTPase-activating protein and VPS9 domain-containing protein 1"
}